6-pyruvoyltetrahydropterin synthase activity [GO:0003874] (molecular function) Definition: Catalysis of the reaction: 7,8-dihydroneopterin 3'-triphosphate = 6-pyruvoyl-5,6,7,8-tetrahydropterin + H+ + triphosphate. Also known as: 2-amino-4-oxo-6-[(1S,2R)-1,2-dihydroxy-3-triphosphooxypropyl]-7,8-dihydroxypteridine triphosphate lyase activity, 2-amino-4-oxo-6-[(1S,2R)-1,2-dihydroxy-3-triphosphooxypropyl]-7,8-dihydroxypteridine triphosphate-lyase (6-pyruvoyl-5,6,7,8-tetrahydropterin-forming), 6-pyruvoyl tetrahydrobiopterin synthase activity, PTPS activity Relationships: is a type of carbon-oxygen lyase activity, acting on phosphates [GO:0016838] Sources: EC:4.2.3.12, RHEA:22048